{
  "term_id": "GO:0005096",
  "gene_symbol": "TBC1D9",
  "gene_name": "TBC1 domain family member 9",
  "gene": "UniProtKB:Q6ZT07",
  "term_label": "GTPase activator activity"
}